convergent extension involved in gastrulation [GO:0060027] (biological process) Relationships: is a type of embryonic morphogenesis [GO:0048598]; is a type of convergent extension [GO:0060026]; is part of gastrulation [GO:0007369] Regulation: regulated by GO:1904103; negatively regulated by negative regulation of convergent extension involved in gastrulation [GO:1904104]; positively regulated by positive regulation of convergent extension involved in gastrulation [GO:1904105] Subtypes: convergent extension involved in neural plate elongation [GO:0022007], convergent extension involved in somitogenesis [GO:0090246], convergent extension involved in rhombomere morphogenesis [GO:1904125], convergent extension involved in notochord morphogenesis [GO:1904126] Definition: The morphogenetic process in which an epithelium narrows along one axis and lengthens in a perpendicular axis usually resulting in the formation of the three primary germ layers, ectoderm, mesoderm and endoderm. References: PMID:12062082 Sources: GOC:dph